ribitol beta-1,4-xylosyltransferase activity [GO:0120053] (molecular function) Definition: Catalysis of the reaction: UDP-D-xylose + D-ribitol 5-phosphate-R = UDP + beta1,4-xylosyl-D-ribitol 5-phosphate-R. References: PMID:27733679 Relationships: is a type of GO:0035252